{
  "gene_symbol": "SOX3",
  "term_id": "GO:0005634",
  "gene_name": "Transcription factor SOX-3",
  "term_label": "nucleus",
  "gene": "UniProtKB:P41225"
}